integrin alphav-beta8 complex [GO:0034686] (cellular component) Definition: An integrin complex that comprises one alphav subunit and one beta8 subunit. Relationships: is a type of integrin complex [GO:0008305] References: PMID:12297042 Also known as: alphav-beta8 integrin complex, ITGAV-ITGB8 complex